{
  "gene": "UniProtKB:Q96PX8",
  "term_label": "positive regulation of synapse assembly",
  "gene_symbol": "SLITRK1",
  "gene_name": "SLIT and NTRK-like protein 1",
  "term_id": "GO:0051965"
}